2-haloacid dehalogenase (configuration-retaining) activity [GO:0033977] (molecular function) Definition: Catalysis of the reactions: (S)-2-haloacid + H2O = (S)-2-hydroxyacid + halide, and (R)-2-haloacid + H2O = (R)-2-hydroxyacid + halide. Sources: RHEA:12072 Also known as: 2-haloalkanoic acid dehalogenase activity, 2-haloalkanoid acid halidohydrolase activity, DL-2-haloacid dehalogenase activity, DL-DEXr Relationships: is a type of hydrolase activity, acting on acid halide bonds, in C-halide compounds [GO:0019120]